{
  "gene_name": "Protein archease",
  "gene": "UniProtKB:Q8IWT0",
  "gene_symbol": "ZBTB8OS",
  "term_id": "UNKNOWN:0001",
  "term_label": "Unknown molecular function"
}